proton-transporting V-type ATPase complex assembly [GO:0070070] (biological process) Definition: The aggregation, arrangement and bonding together of a proton-transporting V-type ATPase complex, proton-transporting two-sector ATPase complex that couples ATP hydrolysis to the transport of protons across a concentration gradient. Subtypes: vacuolar proton-transporting V-type ATPase complex assembly [GO:0070072] Also known as: V-ATPase assembly, V-ATPase complex assembly Relationships: is a type of GO:0070071 Sources: GOC:mah